{
  "term_label": "spliceosomal complex disassembly",
  "gene_name": "Tuftelin-interacting protein 11",
  "gene_symbol": "TFIP11",
  "term_id": "GO:0000390",
  "gene": "UniProtKB:Q9UBB9"
}